{
  "gene_name": "Semaphorin-3D",
  "gene": "UniProtKB:O95025",
  "term_label": "neuropilin binding",
  "gene_symbol": "SEMA3D",
  "term_id": "GO:0038191"
}